{
  "term_id": "GO:0030280",
  "gene_name": "Keratin, type I cytoskeletal 10",
  "gene": "UniProtKB:P13645",
  "term_label": "structural constituent of skin epidermis",
  "gene_symbol": "KRT10"
}